{
  "gene_symbol": "UFC1",
  "term_id": "GO:0061709",
  "gene": "UniProtKB:Q9Y3C8",
  "gene_name": "Ubiquitin-fold modifier-conjugating enzyme 1",
  "term_label": "reticulophagy"
}